{
  "term_label": "Unknown cellular component",
  "gene_symbol": "IGHD3-10",
  "gene": "UniProtKB:A0A0J9YXN1",
  "term_id": "UNKNOWN:0003",
  "gene_name": "Immunoglobulin heavy diversity 3-10 (Fragment)"
}